{
  "gene": "UniProtKB:Q9UBL9",
  "gene_name": "P2X purinoceptor 2",
  "term_label": "plasma membrane",
  "term_id": "GO:0005886",
  "gene_symbol": "P2RX2"
}